{
  "gene_name": "Androgen-dependent TFPI-regulating protein",
  "gene": "UniProtKB:Q96IZ2",
  "gene_symbol": "ADTRP",
  "term_id": "GO:0012505",
  "term_label": "endomembrane system"
}